{
  "gene": "UniProtKB:Q8TC27",
  "gene_symbol": "ADAM32",
  "term_id": "GO:0006508",
  "term_label": "proteolysis",
  "gene_name": "Disintegrin and metalloproteinase domain-containing protein 32"
}